{
  "gene_name": "Histone-lysine N-methyltransferase, H3 lysine-79 specific",
  "term_label": "subtelomeric heterochromatin formation",
  "term_id": "GO:0031509",
  "gene": "UniProtKB:Q8TEK3",
  "gene_symbol": "DOT1L"
}